{
  "gene": "UniProtKB:Q96F63",
  "term_label": "Unknown biological process",
  "term_id": "UNKNOWN:0002",
  "gene_name": "Coiled-coil domain-containing protein 97",
  "gene_symbol": "CCDC97"
}